somatic diversification of immune receptors via somatic mutation [GO:0002566] (biological process) Relationships: is a type of GO:0002200 Definition: The process in which immune receptor genes are diversified through somatic mutation. Subtypes: somatic hypermutation of immunoglobulin genes [GO:0016446] References: PMID:16102575 Sources: ISBN:0781735149